{
  "gene_symbol": "TTC32",
  "term_id": "UNKNOWN:0002",
  "term_label": "Unknown biological process",
  "gene_name": "Tetratricopeptide repeat protein 32",
  "gene": "UniProtKB:Q5I0X7"
}